thrombin-activated receptor activity [GO:0015057] (molecular function) References: PMID:20423334 Sources: GOC:ai, GOC:pg Relationships: is a type of proteinase-activated receptor activity [GO:0001648]; BFO_0000050 thrombin-activated receptor signaling pathway [GO:0070493] Also known as: thrombin receptor activity, thrombin receptor activity, G-protein coupled Definition: A G protein-coupled receptor activity that is activated by cleavage by thrombin, which exposes a tethered ligand corresponding to the new N-terminus, which binds to the receptor and activates it.